lung growth [GO:0060437] (BP) Definition: The increase in size or mass of a lung. In all air-breathing vertebrates the lungs are developed from the ventral wall of the oesophagus as a pouch which divides into two sacs. In amphibians and many reptiles the lungs retain very nearly this primitive sac-like character, but in the higher forms the connection with the esophagus becomes elongated into the windpipe and the inner walls of the sacs become more and more divided, until, in the mammals, the air spaces become minutely divided into tubes ending in small air cells, in the walls of which the blood circulates in a fine network of capillaries. In mammals the lungs are more or less divided into lobes, and each lung occupies a separate cavity in the thorax. Relationships: is_a organ growth [GO:0035265]; is part of GO:0030324 Sources: GOC:dph